peptidyl-lysine butyrylation [GO:0140067] (biological process) Definition: The butyrylation of a lysine residue in a protein. Butyryl is the univalent radical C3H7COO- derived from butyric acid. References: PMID:27105113 Sources: Wikipedia:butyryl Relationships: is a type of protein acylation [GO:0043543]